{
  "gene": "UniProtKB:Q96MK2",
  "term_id": "UNKNOWN:0003",
  "term_label": "Unknown cellular component",
  "gene_symbol": "RIPOR3",
  "gene_name": "RIPOR family member 3"
}